tyrosinase activity [GO:0004503] (molecular function) Note: In mammals, L-DOPA can act as a cofactor for the catalyzed reaction; therefore in some resources L-DOPA is shown on both sides of the reaction. GO:0004503 describes the monooxygenation of the monophenol, L-tyrosine. For oxidation of diphenols (including L-DOPA and dopamine), consider instead the term 'catechol oxidase activity ; GO:0004097' and its children. Relationships: is a type of oxidoreductase activity, acting on paired donors, with incorporation or reduction of molecular oxygen, another compound as one donor, and incorporation of one atom of oxygen [GO:0016716] References: PMID:4965136 Sources: RHEA:18117 Definition: Catalysis of the reaction: L-tyrosine + O2 = L-DOPAquinone + H2O. This reaction can use both monophenols (such as tyrosine) and catechols (o-diphenols) as substrates. Also known as: phenol oxidase activity, phenolase activity, pyrocatechol oxidase, L-tyrosine monooxygenase activity, monophenol monooxygenase activity, monophenol oxygenase, N-acetyl-6-hydroxytryptophan oxidase activity, catecholase, chlorogenic acid oxidase activity, chlorogenic oxidase activity, cresolase activity, dopa oxidase, monophenol monooxidase activity, monophenol oxidase activity, monophenolase activity, o-diphenol oxidase activity, o-diphenol oxidoreductase, o-diphenol:O2 oxidoreductase activity, prophenol oxidase activity, prophenoloxidase activity, tyrosine-dopa oxidase activity